alpha-1,4-glucan glucosyltransferase (NDP-glucose donor) activity [GO:0033840] (molecular function) Subtypes: alpha-1,4-glucan glucosyltransferase (UDP-glucose donor) activity [GO:0004373], alpha-1,4-glucan glucosyltransferase (ADP-glucose donor) activity [GO:0009011] Relationships: is a type of glucosyltransferase activity [GO:0046527] Also known as: GBSS, GBSSI, GBSSII, NDP-glucose:1,4-alpha-D-glucan 4-alpha-D-glucosyltransferase activity, NDPglucose-starch glucosyltransferase activity, granule-bound starch synthase I activity, granule-bound starch synthase II activity, granule-bound starch synthase activity, starch granule-bound nucleoside diphosphate glucose-starch glucosyltransferase activity, starch synthase II activity, waxy protein Definition: Catalysis of the reaction: [(1->4)-alpha-D-glucosyl](n) + an NDP-alpha-D-glucose = [(1->4)-alpha-D-glucosyl](n+1) + a ribonucleoside 5'-diphosphate + H+, where NDP is ADP or UDP. References: PMID:17472966 Sources: EC:2.4.1.242, RHEA:15873